membrane fusion [GO:0061025] (biological process) Also known as: cellular membrane fusion, single-organism membrane fusion Definition: The membrane organization process that joins two lipid bilayers to form a single membrane. Relationships: is a type of membrane organization [GO:0061024] Subtypes: membrane fusion involved in acrosome reaction [GO:0002078], fusion of virus membrane with host plasma membrane [GO:0019064], plasma membrane fusion [GO:0045026], organelle membrane fusion [GO:0090174] Sources: GOC:dph, GOC:tb